{
  "gene": "UniProtKB:Q9NXV2",
  "term_label": "cytoplasm",
  "gene_name": "BTB_POZ domain-containing protein KCTD5",
  "gene_symbol": "KCTD5",
  "term_id": "GO:0005737"
}